{
  "term_label": "Golgi apparatus",
  "term_id": "GO:0005794",
  "gene_name": "Transmembrane emp24 domain-containing protein 6",
  "gene_symbol": "TMED6",
  "gene": "UniProtKB:Q8WW62"
}